{
  "gene": "UniProtKB:Q96FS4",
  "term_label": "Unknown biological process",
  "gene_name": "Signal-induced proliferation-associated protein 1",
  "term_id": "UNKNOWN:0002",
  "gene_symbol": "SIPA1"
}